{
  "term_id": "GO:0050660",
  "gene_symbol": "LDHD",
  "gene": "UniProtKB:Q86WU2",
  "term_label": "flavin adenine dinucleotide binding",
  "gene_name": "Probable D-lactate dehydrogenase, mitochondrial"
}